{
  "gene": "UniProtKB:Q9Y330",
  "term_label": "DNA-binding transcription repressor activity, RNA polymerase II-specific",
  "gene_symbol": "ZBTB12",
  "gene_name": "Zinc finger and BTB domain-containing protein 12",
  "term_id": "GO:0001227"
}